{
  "term_id": "UNKNOWN:0002",
  "term_label": "Unknown biological process",
  "gene_name": "Coenzyme Q-binding protein COQ10 homolog A, mitochondrial",
  "gene": "UniProtKB:Q96MF6",
  "gene_symbol": "COQ10A"
}